{
  "term_id": "GO:0005615",
  "gene": "UniProtKB:Q99784",
  "gene_name": "Noelin",
  "gene_symbol": "OLFM1",
  "term_label": "extracellular space"
}